vesicle-mediated intercellular transport [GO:0110077] (biological process) Also known as: endosomal trafficking References: PMID:29328915, PMID:29328916 Sources: GOC:sp Definition: A cellular transport process in which transported substances are moved in extracellular vesicles between cells; transported substances are enclosed in the vesicle lumen or located in the extracellular vesicle membrane. Relationships: is a type of intercellular transport [GO:0010496]; is a type of vesicle-mediated transport [GO:0016192]